xenobiotic transmembrane transporter activity [GO:0042910] (MF) Relationships: is a type of transmembrane transporter activity [GO:0022857]; is part of xenobiotic transport [GO:0042908] Sources: GOC:go_curators, GOC:krc Also known as: drug transmembrane transporter activity, drug transporter activity, multidrug efflux pump activity, multidrug transporter activity, multidrug, alkane resistant pump activity, xenobiotic transporter activity Subtypes: ABC-type xenobiotic transporter activity [GO:0008559], methotrexate transmembrane transporter activity [GO:0015350], GO:0015638, bacteriocin transmembrane transporter activity [GO:0022885], benzoate transmembrane transporter activity [GO:0042925], 3-hydroxyphenylpropionic acid transmembrane transporter activity [GO:0042926] Definition: Enables the directed movement of a xenobiotic from one side of a membrane to the other. A xenobiotic is a compound foreign to the organism exposed to it. It may be synthesized by another organism (like ampicilin) or it can be a synthetic chemical.